{
  "gene_symbol": "ST8SIA2",
  "gene_name": "Alpha-2,8-sialyltransferase 8B",
  "gene": "UniProtKB:Q92186",
  "term_label": "oligosaccharide metabolic process",
  "term_id": "GO:0009311"
}